pyruvate dehydrogenase complex [GO:0045254] (CC) Also known as: pyruvate dehydrogenase complex (lipoamide) References: PMID:36863425 Relationships: is a type of alpha-ketoacid dehydrogenase complex [GO:0045240]; is a type of GO:1902493 Note: The catalytic activities of the individual components of this complex are represented by the molecular function terms 'pyruvate dehydrogenase (acetyl-transferring) activity ; GO:0004739' (E1), 'dihydrolipoyllysine-residue acetyltransferase activity ; GO:0004742' (E2), and 'dihydrolipoyl dehydrogenase activity ; GO:0004148' (E3). Definition: A multi-enzyme complex that catalyzes the oxidative decarboxylation of pyruvate to form acetyl-CoA. The complex comprises multiple copies of three enzymes referred to as E1, E2 and E3: pyruvate dehydrogenase (E1, which may be a homodimer or a heterotetramer of two alpha and two beta subunits, depending on species), dihydrolipoamide S-acetyltransferase (E2), and dihydrolipoamide dehydrogenase (E3). Additional proteins may also be present.